{
  "gene": "UniProtKB:O60936",
  "gene_symbol": "NOL3",
  "term_label": "death receptor binding",
  "term_id": "GO:0005123",
  "gene_name": "Nucleolar protein 3"
}